acetaldehyde dehydrogenase (NAD+) activity [GO:0140087] (molecular function) References: PMID:9473035 Sources: RHEA:25294 Definition: Catalysis of the reaction: acetaldehyde + NAD+ + H2O = acetate + NADH + 2 H+. Relationships: is a type of aldehyde dehydrogenase (NAD+) activity [GO:0004029]